{
  "term_label": "nucleoplasm",
  "gene_name": "Heterogeneous nuclear ribonucleoprotein H2",
  "gene": "UniProtKB:P55795",
  "gene_symbol": "HNRNPH2",
  "term_id": "GO:0005654"
}